medium-chain fatty-acyl-CoA catabolic process [GO:0036114] (biological process) Relationships: is a type of medium-chain fatty-acyl-CoA metabolic process [GO:0036112]; is a type of fatty-acyl-CoA catabolic process [GO:0036115] Note: While there is not universal consensus on the lengths of short-, medium-, long- and very-long-chain fatty acids, the GO uses the definitions in ChEBI (see CHEBI:26666, CHEBI:59554, CHEBI:15904 and CHEBI:27283). Also known as: medium-chain fatty-acyl-CoA breakdown, medium-chain fatty-acyl-CoA catabolism, medium-chain fatty-acyl-CoA degradation Sources: GOC:pm Definition: The chemical reactions and pathways resulting in the breakdown of medium-chain fatty-acyl-CoAs, any derivative of coenzyme A in which the sulfhydryl group is in a thioester linkage with a medium-chain fatty-acyl group. A medium-chain fatty acid has an aliphatic tail containing 6 to 12 carbons.